adrenergic receptor binding [GO:0031690] (molecular function) Definition: Binding to an adrenergic receptor. Sources: GOC:mah, GOC:nln Also known as: adrenergic receptor ligand Relationships: is a type of GO:0001664 Subtypes: alpha-1A adrenergic receptor binding [GO:0031691], alpha-1B adrenergic receptor binding [GO:0031692], alpha-1D adrenergic receptor binding [GO:0031693], alpha-2A adrenergic receptor binding [GO:0031694], alpha-2B adrenergic receptor binding [GO:0031695], alpha-2C adrenergic receptor binding [GO:0031696], GO:0031697, beta-2 adrenergic receptor binding [GO:0031698], beta-3 adrenergic receptor binding [GO:0031699]